peptidyl-proline di-hydroxylation [GO:0018188] (biological process) Relationships: is a type of GO:0019511 Sources: RESID:AA0282 Definition: The modification of peptidyl-proline to form trans-2,3-cis-3,4-dihydroxy-L-proline.